{
  "term_label": "cAMP-dependent protein kinase activity",
  "gene_name": "Putative serine_threonine-protein kinase PRKY",
  "term_id": "GO:0004691",
  "gene_symbol": "PRKY",
  "gene": "UniProtKB:O43930"
}